{
  "term_label": "animal organ morphogenesis",
  "term_id": "GO:0009887",
  "gene_symbol": "NTN4",
  "gene": "UniProtKB:Q9HB63",
  "gene_name": "Netrin-4"
}